{
  "gene_symbol": "CA2",
  "gene": "UniProtKB:P00918",
  "term_id": "GO:0005886",
  "term_label": "plasma membrane",
  "gene_name": "Carbonic anhydrase 2"
}